{
  "term_label": "Unknown biological process",
  "term_id": "UNKNOWN:0002",
  "gene_symbol": "TECTB",
  "gene": "UniProtKB:Q96PL2",
  "gene_name": "Beta-tectorin"
}